RNA polymerase I preinitiation complex assembly [GO:0001188] (biological process) Definition: The formation of a large multiprotein-DNA complex that self-assembles on gene promoter through the sequential recruitment of the general initiation factors that compose the preinitiation complex (PIC) (which includes including UBF, SL1, RRN3 and TBP in human). The PIC engages RNA polymerase I on its DNA template strand and sparks polymerization of the first few RNA nucleotides. Relationships: is a type of GO:0070897; is part of transcription initiation at RNA polymerase I promoter [GO:0006361] References: PMID:14969726 Sources: GOC:txnOH Also known as: RNA polymerase I transcriptional preinitiation complex assembly, RNA polymerase I transcriptional preinitiation complex assembly at the promoter for the nuclear large rRNA transcript, RNA polymerase I transcriptional preinitiation complex assembly at the promoter for the nucleolar primary rRNA transcript